vanadium-iron nitrogenase complex [GO:0016613] (cellular component) Also known as: vanadium-iron nitrogenase activity Relationships: is_a nitrogenase complex [GO:0016610] Definition: An enzyme complex containing a vanadium-iron cluster found in some species, such as Azotobacter vinelandii. It is composed of two proteins, dinitrogenase and nitrogenase reductase; dinitrogenase, the vanadium-iron protein, is tetrameric with an alpha2-beta2 structure, and nitrogenase reductase is a homodimer. References: PMID:3474027